zeaxanthin 2,2'-beta-hydroxylase activity [GO:0102465] (molecular function) Sources: GOC:pz Definition: Catalysis of the reaction: zeaxanthin + 2 NADH + 2 H+ + 2 O2 = nostoxanthin + 2 NAD + 2 H2O. Relationships: is a type of GO:0016709